{
  "gene": "UniProtKB:P41002",
  "gene_symbol": "CCNF",
  "gene_name": "Cyclin-F",
  "term_id": "GO:0005737",
  "term_label": "cytoplasm"
}